positive regulation of lysosome organization [GO:1905673] (BP) Relationships: is a type of positive regulation of vacuole organization [GO:0044090]; is a type of regulation of lysosome organization [GO:1905671]; positively regulates lysosome organization [GO:0007040] Also known as: positive regulation of lysosome organisation, up regulation of lysosome organisation, up regulation of lysosome organization, up-regulation of lysosome organisation, up-regulation of lysosome organization, upregulation of lysosome organisation, upregulation of lysosome organization, activation of lysosome organisation, activation of lysosome organization, activation of lysosome organization and biogenesis, positive regulation of lysosome organization and biogenesis, up regulation of lysosome organization and biogenesis, up-regulation of lysosome organization and biogenesis, upregulation of lysosome organization and biogenesis Definition: Any process that activates or increases the frequency, rate or extent of lysosome organization. References: PMID:25561470 Sources: GOC:TermGenie, GO_REF:0000058